{
  "gene_symbol": "OR7A17",
  "gene_name": "Olfactory receptor 7A17",
  "term_id": "GO:0004984",
  "gene": "UniProtKB:O14581",
  "term_label": "olfactory receptor activity"
}